{
  "term_label": "Unknown biological process",
  "gene_name": "Nuclear pore complex-interacting protein family member A5",
  "gene_symbol": "NPIPA5",
  "gene": "UniProtKB:E9PKD4",
  "term_id": "UNKNOWN:0002"
}